{
  "gene_symbol": "PI15",
  "gene_name": "Peptidase inhibitor 15",
  "term_id": "UNKNOWN:0002",
  "term_label": "Unknown biological process",
  "gene": "UniProtKB:O43692"
}